{
  "term_label": "sodium ion transmembrane transport",
  "term_id": "GO:0035725",
  "gene_name": "Sodium channel protein type 8 subunit alpha",
  "gene": "UniProtKB:Q9UQD0",
  "gene_symbol": "SCN8A"
}